{
  "gene": "UniProtKB:Q9NRD8",
  "term_label": "NADPH oxidase complex",
  "gene_name": "Dual oxidase 2",
  "term_id": "GO:0043020",
  "gene_symbol": "DUOX2"
}